{
  "gene_name": "Baculoviral IAP repeat-containing protein 3",
  "gene": "UniProtKB:Q13489",
  "gene_symbol": "BIRC3",
  "term_id": "GO:0043027",
  "term_label": "cysteine-type endopeptidase inhibitor activity involved in apoptotic process"
}